{
  "gene": "UniProtKB:O94993",
  "term_id": "GO:0006357",
  "term_label": "regulation of transcription by RNA polymerase II",
  "gene_symbol": "SOX30",
  "gene_name": "Transcription factor SOX-30"
}